mitotic actomyosin contractile ring maturation [GO:1902406] (biological process) Definition: The cellular process in which the mitotic contractile ring cytokinetic ring attains its fully functional state. References: PMID:25451933 Relationships: is a type of actomyosin contractile ring maturation [GO:0031566]; is a type of GO:1903047; is part of mitotic cytokinesis [GO:0000281] Also known as: mitotic cytokinesis contractile ring maintenance